negative regulation of cell projection organization [GO:0031345] (biological process) Subtypes: negative regulation of axonemal microtubule depolymerization [GO:0007027], negative regulation of neuron projection development [GO:0010977], negative regulation of dendrite morphogenesis [GO:0050774], GO:0120033, GO:0150013, negative regulation of bacterial-type flagellum assembly [GO:1902209], negative regulation of lamellipodium organization [GO:1902744], negative regulation of dendritic spine maintenance [GO:1902951], negative regulation of type IV pilus biogenesis [GO:1903657], negative regulation of microvillus length [GO:1903982] Sources: GOC:mah Also known as: down regulation of cell projection organization, down-regulation of cell projection organization, downregulation of cell projection organization, negative regulation of cell projection organisation, inhibition of cell projection organization, negative regulation of cell projection organization and biogenesis Definition: Any process that stops, prevents, or reduces the frequency, rate or extent of a process involved in the formation, arrangement of constituent parts, or disassembly of cell projections. Relationships: is a type of regulation of cell projection organization [GO:0031344]; is a type of GO:0051129; negatively regulates cell projection organization [GO:0030030]